collateral sprouting in absence of injury [GO:0048669] (biological process) Regulation: regulated by GO:0048696; positively regulated by positive regulation of collateral sprouting in absence of injury [GO:0048697]; RO_0002212 by negative regulation of collateral sprouting in absence of injury [GO:0048698] Definition: The process in which outgrowths develop from the axons of intact undamaged neurons. Sources: GOC:dgh, GOC:dph, GOC:jid, GOC:lm Relationships: is a type of collateral sprouting [GO:0048668]